{
  "term_label": "plasma membrane",
  "gene_symbol": "PALS2",
  "gene_name": "Protein PALS2",
  "gene": "UniProtKB:Q9NZW5",
  "term_id": "GO:0005886"
}